neurotransmitter transport [GO:0006836] (biological process) Subtypes: neurotransmitter uptake [GO:0001504], GO:0007269, neurotransmitter loading into synaptic vesicle [GO:0098700] Regulation: regulated by regulation of neurotransmitter transport [GO:0051588]; negatively regulated by GO:0051589; positively regulated by positive regulation of neurotransmitter transport [GO:0051590] Relationships: is a type of transport [GO:0006810] Sources: GOC:ai Definition: The directed movement of a neurotransmitter into, out of or within a cell, or between cells, by means of some agent such as a transporter or pore. Neurotransmitters are any chemical substance that is capable of transmitting (or inhibiting the transmission of) a nerve impulse from a neuron to another cell. Also known as: sodium:neurotransmitter transport